{
  "term_id": "GO:0061630",
  "gene": "UniProtKB:Q8ND25",
  "gene_name": "E3 ubiquitin-protein ligase ZNRF1",
  "gene_symbol": "ZNRF1",
  "term_label": "ubiquitin protein ligase activity"
}